{
  "gene_name": "Serine_threonine-protein kinase LMTK1",
  "term_id": "GO:0051402",
  "gene": "UniProtKB:Q6ZMQ8",
  "gene_symbol": "AATK",
  "term_label": "neuron apoptotic process"
}